{
  "gene_symbol": "LIME1",
  "term_id": "GO:0050853",
  "gene": "UniProtKB:Q9H400",
  "gene_name": "Lck-interacting transmembrane adapter 1",
  "term_label": "B cell receptor signaling pathway"
}